{
  "gene_symbol": "CDY2A",
  "gene_name": "Testis-specific chromodomain protein Y 2",
  "gene": "UniProtKB:Q9Y6F7",
  "term_id": "GO:0120094",
  "term_label": "negative regulation of peptidyl-lysine crotonylation"
}